L-arginine biosynthetic process [GO:0006526] (biological process) Regulation: regulated by GO:1900079; positively regulated by positive regulation of arginine biosynthetic process [GO:1900080] Subtypes: L-arginine biosynthetic process via ornithine [GO:0042450], GO:0170067 Also known as: arginine anabolism, arginine biosynthesis, arginine formation, arginine synthesis Definition: The chemical reactions and pathways resulting in the formation of arginine, 2-amino-5-(carbamimidamido)pentanoic acid. Sources: ISBN:0198506732 Relationships: is a type of arginine metabolic process [GO:0006525]; is_a glutamine family amino acid biosynthetic process [GO:0009084]